acetylxylan esterase activity [GO:0046555] (molecular function) Sources: EC:3.1.1.72 Definition: Catalysis of the deacetylation of xylans and xylo-oligosaccharides. Relationships: is a type of carboxylic ester hydrolase activity [GO:0052689]